itaconyl-CoA hydratase activity [GO:0050011] (MF) Relationships: is a type of hydro-lyase activity [GO:0016836] Also known as: citramalyl-CoA hydro-lyase (itaconyl-CoA-forming), citramalyl-CoA hydro-lyase activity, itaconyl coenzyme A hydratase activity Sources: EC:4.2.1.56, MetaCyc:ITACONYL-COA-HYDRATASE-RXN Definition: Catalysis of the reaction: citramalyl-CoA = itaconyl-CoA + H2O.